regulation of defense response to virus [GO:0050688] (biological process) Definition: Any process that modulates the frequency, rate or extent of the antiviral response of a cell or organism. Subtypes: negative regulation of defense response to virus [GO:0050687], regulation of defense response to virus by host [GO:0050691] Sources: GOC:ai Relationships: is a type of regulation of response to biotic stimulus [GO:0002831]; is a type of GO:0031347; is a type of GO:0032101; regulates defense response to virus [GO:0051607] Also known as: regulation of antiviral response